{
  "term_label": "Unknown molecular function",
  "gene_name": "Cadherin EGF LAG seven-pass G-type receptor 2",
  "gene_symbol": "CELSR2",
  "gene": "UniProtKB:Q9HCU4",
  "term_id": "UNKNOWN:0001"
}